MMXD complex [GO:0071817] (cellular component) Also known as: MMS19-MIP18-XPD complex Definition: A protein complex that contains the proteins MMS19, MIP18 and XPD, localizes to mitotic spindle during mitosis, and is required for proper chromosome segregation. References: PMID:20797633 Sources: GOC:sp Relationships: is a type of protein-containing complex [GO:0032991]; is part of spindle [GO:0005819]